positive regulation of biosynthetic process of antibacterial peptides active against Gram-negative bacteria [GO:0006964] (biological process) Relationships: is a type of GO:0002813; is a type of positive regulation of antibacterial peptide biosynthetic process [GO:0006963]; positively regulates biosynthetic process of antibacterial peptides active against Gram-negative bacteria [GO:0002812] Definition: Any process that activates or increases the frequency, rate, or extent of biosynthesis of antibacterial peptides active against Gram-negative bacteria. Also known as: anti-Gram-negative bacterial peptide induction, anti-Gram-negative bacterial polypeptide induction, up regulation of biosynthetic process of antibacterial peptides active against Gram-negative bacteria, up-regulation of biosynthetic process of antibacterial peptides active against Gram-negative bacteria, upregulation of biosynthetic process of antibacterial peptides active against Gram-negative bacteria, activation of biosynthetic process of antibacterial peptides active against Gram-negative bacteria, stimulation of biosynthetic process of antibacterial peptides active against Gram-negative bacteria References: PMID:10973475 Sources: GOC:mah